{
  "gene": "UniProtKB:P10828",
  "term_label": "RNA polymerase II transcription regulator complex",
  "term_id": "GO:0090575",
  "gene_symbol": "THRB",
  "gene_name": "Thyroid hormone receptor beta"
}